response to lipid hydroperoxide [GO:0006982] (biological process) Subtypes: GO:0071449 Relationships: is a type of response to hydroperoxide [GO:0033194]; is a type of response to lipid [GO:0033993] Definition: Any process that results in a change in state or activity of a cell or an organism (in terms of movement, secretion, enzyme production, gene expression, etc.) as a result of a lipid hydroperoxide stimulus. Lipid hydroperoxide is the highly reactive primary oxygenated products of polyunsaturated fatty acids. References: PMID:10944149 Sources: GOC:jl Also known as: response to LHPO